plant-type vacuole lumen [GO:0000330] (cellular component) Definition: The volume enclosed within the vacuolar membrane of a vacuole that retains the same shape regardless of cell cycle phase. An example of this is found in Arabidopsis thaliana. Sources: GOC:krc, GOC:mtg_sensu Relationships: is a type of vacuolar lumen [GO:0005775]; is part of plant-type vacuole [GO:0000325] Also known as: lumen of vacuole with cell cycle-independent morphology Subtypes: protein storage vacuole lumen [GO:0034495]